regulation of asymmetric cell division [GO:0009786] (biological process) Subtypes: negative regulation of asymmetric cell division [GO:0045769], GO:0045770, regulation of male germ-line stem cell asymmetric division [GO:1904838] Definition: Any process that modulates the frequency, rate or extent of asymmetric cell division. Sources: GOC:lr Relationships: is_a regulation of cell division [GO:0051302]; RO_0002211 asymmetric cell division [GO:0008356]